{
  "gene": "UniProtKB:O15225",
  "gene_name": "Putative inactivation escape 1 protein",
  "term_label": "Unknown cellular component",
  "term_id": "UNKNOWN:0003",
  "gene_symbol": "INE1"
}